{
  "gene_name": "DNA polymerase iota",
  "gene": "UniProtKB:Q9UNA4",
  "term_id": "UNKNOWN:0003",
  "gene_symbol": "POLI",
  "term_label": "Unknown cellular component"
}